JUN phosphorylation [GO:0007258] (biological process) Sources: GOC:jl Relationships: is a type of GO:0006468; BFO_0000050 GO:0007254 Definition: The process of introducing a phosphate group into a JUN protein.